neural crest-derived cardiac glial cell development [GO:0060954] (biological process) Sources: GOC:mtg_heart Relationships: is a type of GO:0060952; is part of GO:0060951 Definition: The process aimed at the progression of a neural crest-derived cardiac glial cell over time, from initial commitment of the cell to a specific fate, to the fully functional differentiated cell.